{
  "gene_symbol": "LTBP3",
  "gene": "UniProtKB:Q9NS15",
  "term_label": "extracellular space",
  "term_id": "GO:0005615",
  "gene_name": "Latent-transforming growth factor beta-binding protein 3"
}